{
  "gene_symbol": "TTC5",
  "gene_name": "Tetratricopeptide repeat protein 5",
  "term_label": "Unknown biological process",
  "term_id": "UNKNOWN:0002",
  "gene": "UniProtKB:Q8N0Z6"
}